T-helper 1 type immune response [GO:0042088] (biological process) Definition: An immune response which is associated with resistance to intracellular bacteria, fungi, and protozoa, and pathological conditions such as arthritis, and which is typically orchestrated by the production of particular cytokines by T-helper 1 cells, most notably interferon-gamma, IL-2, and lymphotoxin. Sources: GOC:add, ISBN:0781735149 Also known as: Th1 immune response Relationships: is a type of adaptive immune response based on somatic recombination of immune receptors built from immunoglobulin superfamily domains [GO:0002460] Regulation: RO_0002211 by regulation of T-helper 1 type immune response [GO:0002825]; negatively regulated by negative regulation of T-helper 1 type immune response [GO:0002826]; positively regulated by positive regulation of T-helper 1 type immune response [GO:0002827]